{
  "gene_name": "Olfactory receptor 7C2",
  "term_id": "GO:0005886",
  "gene_symbol": "OR7C2",
  "term_label": "plasma membrane",
  "gene": "UniProtKB:O60412"
}